{
  "gene": "UniProtKB:Q9BZE1",
  "gene_symbol": "MRPL37",
  "term_id": "UNKNOWN:0002",
  "gene_name": "Large ribosomal subunit protein mL37",
  "term_label": "Unknown biological process"
}